{
  "gene_name": "Protein virilizer homolog",
  "gene_symbol": "VIRMA",
  "term_label": "RNA N6-methyladenosine methyltransferase complex",
  "gene": "UniProtKB:Q69YN4",
  "term_id": "GO:0036396"
}